{
  "gene_name": "ATP-dependent RNA helicase DDX55",
  "term_label": "Unknown biological process",
  "gene": "UniProtKB:Q8NHQ9",
  "term_id": "UNKNOWN:0002",
  "gene_symbol": "DDX55"
}